{
  "term_label": "regulation of actin cytoskeleton organization",
  "gene_symbol": "RAC2",
  "term_id": "GO:0032956",
  "gene": "UniProtKB:P15153",
  "gene_name": "Ras-related C3 botulinum toxin substrate 2"
}